{
  "term_label": "Unknown cellular component",
  "term_id": "UNKNOWN:0003",
  "gene": "UniProtKB:A8MUP2",
  "gene_name": "Citrate synthase-lysine N-methyltransferase CSKMT, mitochondrial",
  "gene_symbol": "CSKMT"
}